{
  "gene_symbol": "SLC9A3",
  "term_label": "potassium:proton antiporter activity",
  "gene": "UniProtKB:P48764",
  "gene_name": "Sodium_hydrogen exchanger 3",
  "term_id": "GO:0015386"
}